{
  "gene_name": "Putative butyrophilin subfamily 2 member A3",
  "term_label": "external side of plasma membrane",
  "gene_symbol": "BTN2A3P",
  "term_id": "GO:0009897",
  "gene": "UniProtKB:Q96KV6"
}